{
  "gene": "UniProtKB:Q6ZMR5",
  "term_id": "GO:0005886",
  "term_label": "plasma membrane",
  "gene_name": "Transmembrane protease serine 11A",
  "gene_symbol": "TMPRSS11A"
}